{
  "gene": "UniProtKB:A8MTY0",
  "term_label": "Unknown cellular component",
  "gene_name": "Zinc finger protein 724",
  "term_id": "UNKNOWN:0003",
  "gene_symbol": "ZNF724"
}